filamentous growth of a population of unicellular organisms in response to starvation [GO:0036170] (BP) Relationships: is a type of response to starvation [GO:0042594]; is a type of filamentous growth of a population of unicellular organisms [GO:0044182] Regulation: regulated by regulation of filamentous growth of a population of unicellular organisms in response to starvation [GO:1900434]; positively regulated by positive regulation of filamentous growth of a population of unicellular organisms in response to starvation [GO:1900436] References: PMID:17554048 Sources: GOC:di Definition: The process in which a group of unicellular organisms grow in a threadlike, filamentous shape in response to deprivation of nourishment.